plasma lipoprotein particle organization [GO:0071827] (biological process) Also known as: plasma lipoprotein particle organisation Definition: A protein-lipid complex subunit organization process that results in the formation, disassembly, or alteration of a plasma lipoprotein particle. A plasma lipoprotein particle is a spherical particle with a hydrophobic core of triglycerides and/or cholesterol esters, surrounded by an amphipathic monolayer of phospholipids, cholesterol and apolipoproteins. Relationships: is a type of multicellular organismal process [GO:0032501]; is a type of GO:0071825 Sources: GOC:BHF, GOC:mah Subtypes: plasma lipoprotein particle remodeling [GO:0034369], GO:0034377, GO:0071829